venom-mediated perturbation of nervous system process [GO:0140136] (biological process) Relationships: is a type of venom-mediated perturbation of biological process [GO:0035738] Sources: GOC:pg Definition: A process in which an organism alters or subverts a nervous system process in another organism via the action of a venom. Subtypes: venom-mediated perturbation of transmission of nerve impulse [GO:0044487], GO:0044616, venom-mediated suppression of sensory perception of pain [GO:0044741], venom-mediated increase of sensory perception of pain [GO:0044742]